chemoattraction of axon [GO:0061642] (biological process) Definition: The process in which a neuron growth cone is directed to a specific target site in response to an attractive chemical signal. Sources: GOC:dph, GOC:krc Subtypes: chemoattraction of branchiomotor axon [GO:0021792], chemoattraction of dopaminergic neuron axon [GO:0036516], chemoattraction of serotonergic neuron axon [GO:0036517] Relationships: is a type of positive chemotaxis [GO:0050918]; is part of axon guidance [GO:0007411]; is part of cellular response to chemical stimulus [GO:0070887]